{
  "gene": "UniProtKB:D6RA61",
  "gene_symbol": "USP17L22",
  "term_label": "cytosol",
  "term_id": "GO:0005829",
  "gene_name": "Ubiquitin carboxyl-terminal hydrolase 17-like protein 22"
}